{
  "gene_symbol": "C12orf50",
  "term_id": "GO:0005634",
  "term_label": "nucleus",
  "gene": "UniProtKB:Q8NA57",
  "gene_name": "Uncharacterized protein C12orf50"
}